{
  "gene_name": "Histone H2A type 1-B_E",
  "gene": "UniProtKB:P04908",
  "term_id": "GO:0000786",
  "gene_symbol": "H2AC8",
  "term_label": "nucleosome"
}